{
  "term_id": "GO:0032968",
  "term_label": "positive regulation of transcription elongation by RNA polymerase II",
  "gene_name": "RNA polymerase II elongation factor ELL",
  "gene": "UniProtKB:P55199",
  "gene_symbol": "ELL"
}